{
  "gene_name": "Semaphorin-6D",
  "term_label": "chemorepellent activity",
  "gene": "UniProtKB:Q8NFY4",
  "gene_symbol": "SEMA6D",
  "term_id": "GO:0045499"
}